necroptotic signaling pathway [GO:0097527] (biological process) Definition: The series of molecular signals which triggers the necroptotic death of a cell. The pathway starts with reception of a signal, is characterized by activation of receptor-interacting serine/threonine-protein kinase 1 and/or 3 (RIPK1/3, also called RIP1/3), and ends when the execution phase of necroptosis is triggered. References: PMID:20823910 Sources: GOC:mtg_apoptosis Also known as: necroptosis signaling pathway, necroptotic signal transduction, necroptosis signaling, necroptotic signalling pathway Note: Gene products that may be annotated to this term include: 1) ligands such as TNF-alpha; 2) receptors such as TNFR (though care should be taken because TNF-alpha and TNFR may also be involved in non-necroptotic processes); 3) signaling molecules such as TNFR-associated death domain (TRADD), receptor-interacting protein kinase 1 (RIP1), cellular inhibitor of apoptosis 1 (cIAP1), cIAP2, TNFR-associated factor 2 (TRAF2) and TRAF5. Within the so-called complex I, RIP1 is polyubiquitinated by cIAPs, thereby providing a docking site for the recruitment of transforming growth factor beta (TGFbeta)-activated kinase 1 (TAK1), TAK1-binding protein 2 (TAB2) and TAB3 (which together deliver a pro-survival signal by activating the transcription factor NF-kB). In some pathophysiological and experimental settings, and in particular when caspase-8 is absent or when caspases are inhibited by pharmacological agents, cylindromatosis (CYLD)-deubiquitinated RIP1 engage in physical and functional interactions with its homolog RIP3, ultimately activating the execution of necrotic cell death. (The pathway downstream of RIPK3 remains largely unknown, although ROS generation, calcium overload, and the opening of the mitochondrial permeability transition pore have been implicated (PMID:22265414)). A necroptotic signaling pathway may also be induced by alkylating DNA damage (possibly by the overactivation of poly(ADP-ribose) polymerase 1, PARP1). This is sometimes referred to as PARP-dependent cell death or parthanatos; it is still being debated if it constitutes an independent cell death modality. Relationships: is a type of signal transduction [GO:0007165]; is part of necroptotic process [GO:0070266]